negative regulation of macromolecule metabolic process [GO:0010605] (biological process) Relationships: is_a GO:0009892; is a type of regulation of macromolecule metabolic process [GO:0060255]; RO_0002212 macromolecule metabolic process [GO:0043170] Definition: Any process that decreases the frequency, rate or extent of the chemical reactions and pathways involving macromolecules, any molecule of high relative molecular mass, the structure of which essentially comprises the multiple repetition of units derived, actually or conceptually, from molecules of low relative molecular mass. Subtypes: GO:0001920, GO:0010558, GO:0051053, negative regulation of protein metabolic process [GO:0051248], negative regulation of RNA metabolic process [GO:0051253], negative regulation of glycogen metabolic process [GO:0070874], negative regulation of receptor catabolic process [GO:2000645], negative regulation of starch catabolic process [GO:2000882], negative regulation of glucomannan catabolic process [GO:2000907], negative regulation of galactoglucomannan catabolic process [GO:2000913], negative regulation of cellodextrin catabolic process [GO:2000928], negative regulation of cyclodextrin catabolic process [GO:2000958], negative regulation of cell wall polysaccharide catabolic process [GO:2000967], negative regulation of hemicellulose catabolic process [GO:2000989], negative regulation of galactomannan catabolic process [GO:2000992], negative regulation of cellulose catabolic process [GO:2000998], negative regulation of pectin catabolic process [GO:2001004] Sources: GOC:dph, GOC:tb